uroporphyrinogen decarboxylase activity [GO:0004853] (molecular function) Definition: Catalysis of the reaction: uroporphyrinogen-III = coproporphyrinogen + 4 CO2. Sources: EC:4.1.1.37 Also known as: porphyrinogen carboxy-lyase activity, porphyrinogen decarboxylase activity, uroporphyrinogen III decarboxylase activity, uroporphyrinogen-III carboxy-lyase (coproporphyrinogen-III-forming), uroporphyrinogen-III carboxy-lyase activity Relationships: is a type of GO:0016831